glomerular epithelial cell differentiation [GO:0072311] (biological process) Subtypes: mesonephric glomerular epithelial cell differentiation [GO:0061250], podocyte differentiation [GO:0072112], glomerular parietal epithelial cell differentiation [GO:0072139], metanephric glomerular epithelial cell differentiation [GO:0072312] Definition: The process in which a relatively unspecialized cell acquires specialized features of a glomerular epithelial cell. Glomerular epithelial cells are specialized epithelial cells that form part of the glomerulus; there are two types, glomerular parietal epithelial cells and glomerular visceral epithelial cells. Relationships: is a type of epithelial cell differentiation involved in kidney development [GO:0035850]; is part of GO:0072010 Sources: GOC:mtg_kidney_jan10